{
  "term_label": "1-phosphatidylinositol binding",
  "gene_name": "Early endosome antigen 1",
  "term_id": "GO:0005545",
  "gene": "UniProtKB:Q15075",
  "gene_symbol": "EEA1"
}